L-lysine catabolic process to acetyl-CoA via L-pipecolate [GO:0033514] (biological process) Definition: The chemical reactions and pathways resulting in the breakdown of L-lysine into other compounds, including acetyl-CoA, via the intermediate L-pipecolate. Sources: GOC:mah, MetaCyc:PWY-5283 Also known as: L-lysine breakdown to acetyl-CoA via L-pipecolate, L-lysine degradation to acetyl-CoA via L-pipecolate Relationships: is a type of GO:0019474